{
  "term_id": "GO:0060070",
  "gene_symbol": "BCL9L",
  "term_label": "canonical Wnt signaling pathway",
  "gene_name": "B-cell CLL_lymphoma 9-like protein",
  "gene": "UniProtKB:Q86UU0"
}